{
  "gene_symbol": "PTPRF",
  "gene_name": "Receptor-type tyrosine-protein phosphatase F",
  "term_label": "signal transduction",
  "term_id": "GO:0007165",
  "gene": "UniProtKB:P10586"
}